{
  "gene_name": "Cadherin-related family member 3",
  "gene_symbol": "CDHR3",
  "gene": "UniProtKB:Q6ZTQ4",
  "term_id": "GO:0044331",
  "term_label": "cell-cell adhesion mediated by cadherin"
}